{
  "term_label": "MAP kinase tyrosine/serine/threonine phosphatase activity",
  "term_id": "GO:0017017",
  "gene": "UniProtKB:Q13202",
  "gene_name": "Dual specificity protein phosphatase 8",
  "gene_symbol": "DUSP8"
}